{
  "gene_symbol": "HSPA1B",
  "term_id": "GO:0005737",
  "gene": "UniProtKB:P0DMV9",
  "gene_name": "Heat shock 70 kDa protein 1B",
  "term_label": "cytoplasm"
}